{
  "gene": "UniProtKB:Q86Y01",
  "term_id": "GO:0007219",
  "term_label": "Notch signaling pathway",
  "gene_symbol": "DTX1",
  "gene_name": "E3 ubiquitin-protein ligase DTX1"
}